{
  "gene": "UniProtKB:Q9Y239",
  "term_label": "cytosol",
  "gene_name": "Nucleotide-binding oligomerization domain-containing protein 1",
  "term_id": "GO:0005829",
  "gene_symbol": "NOD1"
}